single-celled organism vegetative growth phase [GO:0072690] (biological process) Also known as: vegetative growth of a single-celled organism, stationary phase Relationships: is a type of biological phase [GO:0044848] Sources: GOC:mah, GOV:vw Definition: A phase of population growth during which single celled organisms reproduce by budding, fission, or other asexual methods. Note: Note that this term should not be used for direct annotation. If you are trying to make an annotation to x phase, it is likely that the correct annotation is 'regulation of x/y phase transition' or to a process which occurs during the reported phase. To capture the phase when a specific location or process is observed, the phase term can be used in an annotation extension (PMID:24885854) applied to a cellular component term (with the relation exists_during) or a biological process term (with the relation happens_during).